{
  "gene": "UniProtKB:Q96PY0",
  "term_id": "UNKNOWN:0003",
  "gene_symbol": "PSMG3-AS1",
  "gene_name": "Putative uncharacterized protein PSMG3-AS1",
  "term_label": "Unknown cellular component"
}